{
  "gene": "UniProtKB:Q9BVW5",
  "gene_name": "TIMELESS-interacting protein",
  "term_id": "GO:0003677",
  "term_label": "DNA binding",
  "gene_symbol": "TIPIN"
}